{
  "gene_symbol": "CRNKL1",
  "gene_name": "Crooked neck-like protein 1",
  "term_label": "Prp19 complex",
  "term_id": "GO:0000974",
  "gene": "UniProtKB:Q9BZJ0"
}